{
  "gene_name": "Zinc finger protein 692",
  "term_id": "UNKNOWN:0003",
  "gene_symbol": "ZNF692",
  "gene": "UniProtKB:Q9BU19",
  "term_label": "Unknown cellular component"
}